{
  "term_label": "Unknown biological process",
  "term_id": "UNKNOWN:0002",
  "gene_symbol": "MAMDC2",
  "gene": "UniProtKB:Q7Z304",
  "gene_name": "MAM domain-containing protein 2"
}